{
  "gene": "UniProtKB:P57082",
  "gene_symbol": "TBX4",
  "term_label": "regulation of transcription by RNA polymerase II",
  "gene_name": "T-box transcription factor TBX4",
  "term_id": "GO:0006357"
}